{
  "gene": "UniProtKB:P08173",
  "gene_symbol": "CHRM4",
  "term_label": "G protein-coupled acetylcholine receptor activity",
  "term_id": "GO:0016907",
  "gene_name": "Muscarinic acetylcholine receptor M4"
}